{
  "term_label": "Unknown cellular component",
  "gene_name": "Keratin-associated protein 1-3",
  "gene": "UniProtKB:Q8IUG1",
  "term_id": "UNKNOWN:0003",
  "gene_symbol": "KRTAP1-3"
}